paromomycin biosynthetic process [GO:1901155] (biological process) Definition: The chemical reactions and pathways resulting in the formation of paromomycin. Relationships: is a type of aminoglycoside antibiotic biosynthetic process [GO:0030648]; is a type of polyol biosynthetic process [GO:0046173] Also known as: paromomycin anabolism, paromomycin biosynthesis, paromomycin formation, paromomycin synthesis Sources: GOC:TermGenie, GOC:yaf, UniPathway:UPA00970